{
  "term_id": "UNKNOWN:0001",
  "gene_symbol": "KRTAP1-5",
  "gene": "UniProtKB:Q9BYS1",
  "gene_name": "Keratin-associated protein 1-5",
  "term_label": "Unknown molecular function"
}